{
  "term_label": "membrane",
  "gene": "UniProtKB:Q8WVN6",
  "gene_symbol": "SECTM1",
  "gene_name": "Secreted and transmembrane protein 1",
  "term_id": "GO:0016020"
}